{
  "gene_symbol": "OR52E8",
  "term_label": "plasma membrane",
  "term_id": "GO:0005886",
  "gene": "UniProtKB:Q6IFG1",
  "gene_name": "Olfactory receptor 52E8"
}